icosanoid binding [GO:0050542] (molecular function) Relationships: is a type of GO:0031406 Also known as: eicosanoid binding Subtypes: GO:0050544, GO:0050646, GO:0050647, 5(S)-hydroxyperoxy-6E,8Z,11Z,14Z-icosatetraenoic acid binding [GO:0050648] Definition: Binding to icosanoids, any C20 polyunsaturated fatty acids or their derivatives, including the leukotrienes and the prostanoids. Sources: ISBN:0198506732